{
  "gene_name": "Protein hinderin",
  "term_id": "UNKNOWN:0002",
  "gene": "UniProtKB:Q86T90",
  "term_label": "Unknown biological process",
  "gene_symbol": "KIAA1328"
}